{
  "term_id": "GO:0000981",
  "gene_name": "Zinc finger protein 248",
  "gene": "UniProtKB:Q8NDW4",
  "term_label": "DNA-binding transcription factor activity, RNA polymerase II-specific",
  "gene_symbol": "ZNF248"
}